{
  "gene": "UniProtKB:O00463",
  "gene_symbol": "TRAF5",
  "term_id": "GO:0005737",
  "gene_name": "TNF receptor-associated factor 5",
  "term_label": "cytoplasm"
}